{
  "gene": "UniProtKB:Q0VD83",
  "term_id": "GO:0006641",
  "term_label": "triglyceride metabolic process",
  "gene_symbol": "APOBR",
  "gene_name": "Apolipoprotein B receptor"
}